{
  "gene_name": "Placenta growth factor",
  "gene": "UniProtKB:P49763",
  "gene_symbol": "PGF",
  "term_label": "vascular endothelial growth factor signaling pathway",
  "term_id": "GO:0038084"
}